symbiont-mediated suppression of host interferon-mediated signaling pathway [GO:0140886] (biological process) Subtypes: GO:0039502, symbiont-mediated suppression of host type II interferon-mediated signaling pathway [GO:0140884], symbiont-mediated suppression of host type III interferon-mediated signaling pathway [GO:0140885] References: PMID:31266861, PMID:33097660, PMID:34305858 Relationships: is a type of symbiont-mediated suppression of host signal transduction pathway [GO:0052029] Also known as: suppression by symbiont of host IFN-mediated signaling pathway, suppression by symbiont of host interferon-mediated signalling pathway, negative regulation by virus of host interferon-mediated signaling pathway, suppression by virus of host interferon-mediated signaling pathway, inhibition of host interferon signaling pathway by symbiont Definition: Any process in which a virus stops, prevents, or reduces the frequency, rate or extent of interferon-mediated signaling in the host organism.